{
  "gene": "UniProtKB:Q9UKF6",
  "gene_symbol": "CPSF3",
  "gene_name": "Cleavage and polyadenylation specificity factor subunit 3",
  "term_id": "GO:0003723",
  "term_label": "RNA binding"
}